{
  "gene_name": "S-methyl-5'-thioadenosine phosphorylase",
  "term_id": "GO:0005829",
  "gene": "UniProtKB:Q13126",
  "term_label": "cytosol",
  "gene_symbol": "MTAP"
}